{
  "gene_name": "Glucose-6-phosphate exchanger SLC37A4",
  "term_id": "GO:0061513",
  "term_label": "glucose 6-phosphate:phosphate antiporter activity",
  "gene": "UniProtKB:O43826",
  "gene_symbol": "SLC37A4"
}